{
  "gene_name": "Actin-like protein 6B",
  "term_id": "GO:0003682",
  "term_label": "chromatin binding",
  "gene_symbol": "ACTL6B",
  "gene": "UniProtKB:O94805"
}